protein localization to secretory granule [GO:0033366] (biological process) Relationships: is a type of GO:0033365 Also known as: protein localisation in secretory granule, protein localization in secretory granule Definition: A process in which a protein is transported to, or maintained in, a location within a secretory granule. Subtypes: protein localization to mast cell secretory granule [GO:0033367], GO:0033374 Sources: GOC:mah